{
  "gene_symbol": "KCNJ1",
  "term_id": "GO:1990573",
  "gene": "UniProtKB:P48048",
  "term_label": "potassium ion import across plasma membrane",
  "gene_name": "ATP-sensitive inward rectifier potassium channel 1"
}